positive regulation of protein polymerization [GO:0032273] (biological process) Subtypes: positive regulation of actin filament polymerization [GO:0030838], GO:0030841, GO:0031116, positive regulation of free ubiquitin chain polymerization [GO:1904544] Sources: GOC:mah Also known as: up regulation of protein polymerization, up-regulation of protein polymerization, upregulation of protein polymerization, activation of protein polymerization, stimulation of protein polymerization Definition: Any process that activates or increases the frequency, rate or extent of the process of creating protein polymers. Relationships: is a type of positive regulation of protein-containing complex assembly [GO:0031334]; is a type of regulation of protein polymerization [GO:0032271]; positively regulates protein polymerization [GO:0051258]